{
  "term_label": "negative regulation of BMP signaling pathway",
  "gene_name": "Spartin",
  "gene_symbol": "SPART",
  "gene": "UniProtKB:Q8N0X7",
  "term_id": "GO:0030514"
}